{
  "gene_symbol": "MAP3K5",
  "gene_name": "Mitogen-activated protein kinase kinase kinase 5",
  "term_label": "Unknown cellular component",
  "term_id": "UNKNOWN:0003",
  "gene": "UniProtKB:Q99683"
}